primary branching, open tracheal system [GO:0007428] (biological process) Also known as: primary tracheal branching Relationships: is a type of branching involved in open tracheal system development [GO:0060446] References: PMID:29844090 Sources: GOC:mtg_sensu Definition: Formation of primary branches in the open tracheal system. These form from small groups of cells that migrate out at specific positions, organizing into tubes as they migrate. An example of this is found in Drosophila melanogaster.